{
  "term_label": "intracellular protein transport",
  "gene_symbol": "RAB5C",
  "term_id": "GO:0006886",
  "gene": "UniProtKB:P51148",
  "gene_name": "Ras-related protein Rab-5C"
}